{
  "term_id": "UNKNOWN:0003",
  "gene": "UniProtKB:Q96NL1",
  "term_label": "Unknown cellular component",
  "gene_symbol": "TMEM74",
  "gene_name": "Transmembrane protein 74"
}